{
  "gene_symbol": "SLC44A4",
  "gene": "UniProtKB:Q53GD3",
  "term_label": "choline transport",
  "gene_name": "Choline transporter-like protein 4",
  "term_id": "GO:0015871"
}